{
  "gene_symbol": "SCNM1",
  "term_id": "GO:0008380",
  "gene_name": "Sodium channel modifier 1",
  "gene": "UniProtKB:Q9BWG6",
  "term_label": "RNA splicing"
}